{
  "gene": "UniProtKB:O14531",
  "gene_symbol": "DPYSL4",
  "term_label": "hydrolase activity, acting on carbon-nitrogen (but not peptide) bonds, in cyclic amides",
  "gene_name": "Dihydropyrimidinase-related protein 4",
  "term_id": "GO:0016812"
}